{
  "gene_name": "Inactive serine_threonine-protein kinase VRK3",
  "gene_symbol": "VRK3",
  "term_id": "GO:0007165",
  "term_label": "signal transduction",
  "gene": "UniProtKB:Q8IV63"
}